{
  "gene": "UniProtKB:Q96DR4",
  "gene_symbol": "STARD4",
  "gene_name": "StAR-related lipid transfer protein 4",
  "term_label": "cholesterol transfer activity",
  "term_id": "GO:0120020"
}